{
  "term_id": "GO:0036444",
  "gene": "UniProtKB:Q8IYU8",
  "term_label": "calcium import into the mitochondrion",
  "gene_symbol": "MICU2",
  "gene_name": "Calcium uptake protein 2, mitochondrial"
}